{
  "gene": "UniProtKB:Q9UGM6",
  "gene_name": "Tryptophan--tRNA ligase, mitochondrial",
  "term_id": "GO:0005739",
  "gene_symbol": "WARS2",
  "term_label": "mitochondrion"
}